calcium ion transmembrane transport via low voltage-gated calcium channel [GO:0090676] (biological process) Also known as: generation of T-type calcium current References: PMID:20371816 Sources: GOC:PARL, GOC:bf Definition: A process in which a calcium ion is transported from one side of a membrane to the other by means of a low voltage-gated calcium channel. Relationships: is a type of calcium ion transmembrane transport [GO:0070588]; has part GO:0008332